{
  "term_id": "GO:0005654",
  "gene_symbol": "MYCT1",
  "term_label": "nucleoplasm",
  "gene_name": "Myc target protein 1",
  "gene": "UniProtKB:Q8N699"
}